{
  "term_id": "GO:0012505",
  "gene_name": "Ras-related protein Rab-23",
  "gene": "UniProtKB:Q9ULC3",
  "gene_symbol": "RAB23",
  "term_label": "endomembrane system"
}